{
  "term_id": "GO:0005783",
  "gene_symbol": "P3H2",
  "gene_name": "Prolyl 3-hydroxylase 2",
  "term_label": "endoplasmic reticulum",
  "gene": "UniProtKB:Q8IVL5"
}